{
  "gene_symbol": "RAB30",
  "term_id": "GO:0005802",
  "gene_name": "Ras-related protein Rab-30",
  "gene": "UniProtKB:Q15771",
  "term_label": "trans-Golgi network"
}